{
  "term_label": "small-subunit processome",
  "gene_symbol": "FBLL1",
  "gene": "UniProtKB:A6NHQ2",
  "term_id": "GO:0032040",
  "gene_name": "rRNA_tRNA 2'-O-methyltransferase fibrillarin-like protein 1"
}